{
  "term_label": "Unknown biological process",
  "gene_name": "F-box and WD repeat domain containing protein 10B",
  "gene": "UniProtKB:O95170",
  "gene_symbol": "FBXW10B",
  "term_id": "UNKNOWN:0002"
}